{
  "gene_name": "Transmembrane protein 256",
  "term_id": "GO:0016020",
  "gene": "UniProtKB:Q8N2U0",
  "gene_symbol": "TMEM256",
  "term_label": "membrane"
}